peptidoglycan transport [GO:0015835] (biological process) Also known as: murein transport Relationships: is a type of nitrogen compound transport [GO:0071705]; is a type of carbohydrate derivative transport [GO:1901264] Definition: The directed movement of peptidoglycans, a class of glycoconjugates found in bacterial cell walls, into, out of or within a cell, or between cells, by means of some agent such as a transporter or pore. Subtypes: lipid-linked peptidoglycan transport [GO:0015836] Sources: GOC:ai